exoribonuclease activator activity [GO:0044692] (molecular function) Definition: Binds to and increases the activity of an exoribonuclease. Relationships: is a type of ribonuclease activator activity [GO:0170054]; positively regulates GO:0004532 References: PMID:22570495 Sources: GOC:rb